{
  "gene_name": "Kallikrein-1",
  "term_label": "zymogen activation",
  "term_id": "GO:0031638",
  "gene_symbol": "KLK1",
  "gene": "UniProtKB:P06870"
}